{
  "term_label": "plasma membrane",
  "gene_name": "Probable non-functional T cell receptor beta variable 7-1",
  "gene_symbol": "TRBV7-1",
  "term_id": "GO:0005886",
  "gene": "UniProtKB:A0A0A6YYK4"
}